{
  "term_id": "GO:0005829",
  "term_label": "cytosol",
  "gene_name": "Formin-like protein 1",
  "gene_symbol": "FMNL1",
  "gene": "UniProtKB:O95466"
}